{
  "term_label": "ciliary basal body",
  "gene_symbol": "NEDD1",
  "term_id": "GO:0036064",
  "gene_name": "Protein NEDD1",
  "gene": "UniProtKB:Q8NHV4"
}